Grb2-Sos complex [GO:0070618] (cellular component) References: PMID:7798267, PMID:8940013 Sources: GOC:mah Definition: A protein complex that contains Grb2 and the guanine nucleotide exchange factor Sos (or an ortholog thereof, such as mSos1), and is involved in linking EGFR activation to the p21-Ras pathway. Relationships: is a type of plasma membrane protein complex [GO:0098797] Also known as: Grb2-mSos1 complex